{
  "gene_symbol": "NFATC1",
  "term_id": "GO:0045944",
  "term_label": "positive regulation of transcription by RNA polymerase II",
  "gene": "UniProtKB:O95644",
  "gene_name": "Nuclear factor of activated T-cells, cytoplasmic 1"
}